positive regulation of antigen processing and presentation [GO:0002579] (biological process) Definition: Any process that activates or increases the frequency, rate, or extent of antigen processing and presentation. Sources: GOC:add Also known as: up regulation of antigen processing and presentation, up-regulation of antigen processing and presentation, upregulation of antigen processing and presentation, activation of antigen processing and presentation, stimulation of antigen processing and presentation Relationships: is a type of regulation of antigen processing and presentation [GO:0002577]; is a type of GO:0002684; positively regulates antigen processing and presentation [GO:0019882] Subtypes: GO:0002582, positive regulation of antigen processing and presentation of peptide antigen [GO:0002585], positive regulation of antigen processing and presentation via MHC class Ib [GO:0002594], GO:0002606, positive regulation of monocyte antigen processing and presentation [GO:0002615], positive regulation of macrophage antigen processing and presentation [GO:0002618], GO:0002621, positive regulation of B cell antigen processing and presentation [GO:0002624], positive regulation of T cell antigen processing and presentation [GO:0002627]